{
  "gene_symbol": "CLN8",
  "gene": "UniProtKB:Q9UBY8",
  "term_label": "lipid homeostasis",
  "gene_name": "Protein CLN8",
  "term_id": "GO:0055088"
}